{
  "term_label": "metaphase chromosome alignment",
  "gene": "UniProtKB:P49454",
  "gene_name": "Centromere protein F",
  "gene_symbol": "CENPF",
  "term_id": "GO:0051310"
}